{
  "term_label": "chemorepellent activity",
  "gene_symbol": "SEMA3D",
  "gene_name": "Semaphorin-3D",
  "gene": "UniProtKB:O95025",
  "term_id": "GO:0045499"
}